{
  "gene_symbol": "ACOT6",
  "term_label": "Unknown cellular component",
  "gene_name": "Acyl-coenzyme A thioesterase 6",
  "term_id": "UNKNOWN:0003",
  "gene": "UniProtKB:Q3I5F7"
}